{
  "gene": "UniProtKB:Q9H6D7",
  "gene_name": "HAUS augmin-like complex subunit 4",
  "term_id": "GO:0007098",
  "term_label": "centrosome cycle",
  "gene_symbol": "HAUS4"
}